{
  "gene": "UniProtKB:Q9UHY7",
  "term_id": "GO:0043874",
  "term_label": "acireductone synthase activity",
  "gene_symbol": "ENOPH1",
  "gene_name": "Enolase-phosphatase E1"
}